{
  "term_label": "membrane",
  "term_id": "GO:0016020",
  "gene": "UniProtKB:Q15311",
  "gene_symbol": "RALBP1",
  "gene_name": "RalA-binding protein 1"
}